{
  "gene_symbol": "SSTR4",
  "gene": "UniProtKB:P31391",
  "gene_name": "Somatostatin receptor type 4",
  "term_label": "cellular response to glucocorticoid stimulus",
  "term_id": "GO:0071385"
}